{
  "term_id": "GO:0005829",
  "gene_symbol": "PHPT1",
  "gene": "UniProtKB:Q9NRX4",
  "term_label": "cytosol",
  "gene_name": "14 kDa phosphohistidine phosphatase"
}